{
  "term_id": "GO:0031462",
  "gene_name": "PRAME family member 4",
  "gene": "UniProtKB:O60810",
  "term_label": "Cul2-RING ubiquitin ligase complex",
  "gene_symbol": "PRAMEF4"
}